{
  "gene": "UniProtKB:Q9Y3D8",
  "term_id": "GO:0004017",
  "gene_name": "Adenylate kinase isoenzyme 6",
  "term_label": "AMP kinase activity",
  "gene_symbol": "AK6"
}